{
  "gene_name": "SLAM family member 5",
  "gene": "UniProtKB:Q9UIB8",
  "term_id": "GO:0006955",
  "term_label": "immune response",
  "gene_symbol": "CD84"
}